{
  "term_label": "plasma membrane",
  "gene": "UniProtKB:P47890",
  "gene_symbol": "OR1G1",
  "gene_name": "Olfactory receptor 1G1",
  "term_id": "GO:0005886"
}